{
  "gene_symbol": "KHDC1L",
  "term_label": "cytoplasm",
  "term_id": "GO:0005737",
  "gene_name": "Putative KHDC1-like protein",
  "gene": "UniProtKB:Q5JSQ8"
}